{
  "term_label": "dystrophin-associated glycoprotein complex",
  "term_id": "GO:0016010",
  "gene_symbol": "SNTA1",
  "gene": "UniProtKB:Q13424",
  "gene_name": "Alpha-1-syntrophin"
}